{
  "term_label": "regulation of synaptic transmission, glutamatergic",
  "gene_name": "Metabotropic glutamate receptor 1",
  "term_id": "GO:0051966",
  "gene": "UniProtKB:Q13255",
  "gene_symbol": "GRM1"
}